detection of mechanical stimulus [GO:0050982] (biological process) Subtypes: baroreceptor detection of arterial stretch [GO:0001981], detection of renal blood flow [GO:0002000], detection of muscle stretch [GO:0035995], GO:0050974 Sources: GOC:ai, GOC:dos Definition: The series of events by which a mechanical stimulus is received and converted into a molecular signal. Relationships: is_a detection of external stimulus [GO:0009581]; is a type of detection of abiotic stimulus [GO:0009582]; is a type of response to mechanical stimulus [GO:0009612]